regulation of synaptic transmission, dopaminergic [GO:0032225] (biological process) Relationships: is a type of modulation of chemical synaptic transmission [GO:0050804]; RO_0002211 synaptic transmission, dopaminergic [GO:0001963] Definition: Any process that modulates the frequency, rate or extent of dopaminergic synaptic transmission, the process of communication from a neuron to another neuron across a synapse using the neurotransmitter dopamine. Sources: GOC:mah Subtypes: GO:0032226, negative regulation of synaptic transmission, dopaminergic [GO:0032227]